negative regulation of microtubule polymerization [GO:0031115] (biological process) Sources: GOC:mah Relationships: is a type of negative regulation of microtubule polymerization or depolymerization [GO:0031111]; is a type of regulation of microtubule polymerization [GO:0031113]; is a type of negative regulation of protein polymerization [GO:0032272]; is a type of negative regulation of supramolecular fiber organization [GO:1902904]; negatively regulates GO:0046785 Also known as: down regulation of microtubule polymerization, down-regulation of microtubule polymerization, downregulation of microtubule polymerization, inhibition of microtubule polymerization Definition: Any process that stops, prevents, or reduces the frequency, rate or extent of microtubule polymerization. Subtypes: negative regulation of microtubule nucleation [GO:1905833]